{
  "term_id": "UNKNOWN:0001",
  "gene_name": "Putative uncharacterized protein LINC00574",
  "gene": "UniProtKB:Q9H8X3",
  "term_label": "Unknown molecular function",
  "gene_symbol": "LINC00574"
}